{
  "term_id": "GO:0005737",
  "gene_symbol": "MYL12B",
  "term_label": "cytoplasm",
  "gene_name": "Myosin regulatory light chain 12B",
  "gene": "UniProtKB:O14950"
}